cargo receptor activity [GO:0038024] (molecular function) References: PMID:15239958, PMID:27903609 Subtypes: asialoglycoprotein receptor activity [GO:0004873], transferrin receptor activity [GO:0004998], GO:0005044, vitellogenin receptor activity [GO:0008196], alpha-2 macroglobulin receptor activity [GO:0016964], apolipoprotein receptor activity [GO:0030226], lipoprotein particle receptor activity [GO:0030228], lactoferrin receptor activity [GO:0033568], folic acid receptor activity [GO:0061714], ferritin receptor activity [GO:0070287], COPII receptor activity [GO:0097020], GO:0140488 Relationships: is a type of molecular_function [GO:0003674]; is part of vesicle-mediated transport [GO:0016192]; has part GO:0060090 Also known as: receptor activity, transport receptor activity, endocytic receptor activity, receptor activity involved in receptor-mediated endocytosis Definition: Binding specifically to a substance (cargo) to deliver it to a transport vesicle. Cargo receptors span membranes (for instance the plasma membrane or the endoplasmic reticulum membrane), binding simultaneously to cargo molecules and coat adaptors, to efficiently recruit the cargo molecules to nascent vesicles. Note: Notes: (1) For receptors binding a molecule but coupled to a signal transduction pathway, consider instead the term 'signaling receptor activity ; GO:0038023' and its children. (2) Cargo receptors transport substances by vesicular transport, not by transmembrane transport. For transmembrane transporters, consider instead the term 'transmembrane transporter activity ; GO:0022857'.